{
  "term_label": "centrosome",
  "term_id": "GO:0005813",
  "gene_name": "Kinesin-like protein KIF2B",
  "gene_symbol": "KIF2B",
  "gene": "UniProtKB:Q8N4N8"
}